phosphatidylinositol metabolic process [GO:0046488] (biological process) Relationships: is a type of glycerophospholipid metabolic process [GO:0006650] Subtypes: GPI anchor metabolic process [GO:0006505], phosphatidylinositol biosynthetic process [GO:0006661], phosphatidylinositol catabolic process [GO:0031161], phosphatidylinositol acyl-chain remodeling [GO:0036149], phosphatidylinositol dephosphorylation [GO:0046856], 1-phosphatidyl-1D-myo-inositol 4,5-bisphosphate metabolic process [GO:1902633], 1-phosphatidyl-1D-myo-inositol 3,5-bisphosphate metabolic process [GO:1903100], GO:1904562 Also known as: PtdIns metabolic process, PtdIns metabolism, phosphatidylinositol metabolism, phosphoinositide metabolic process, phosphoinositide metabolism Sources: ISBN:0198506732 Definition: The chemical reactions and pathways involving phosphatidylinositol, any glycophospholipid in which a sn-glycerol 3-phosphate residue is esterified to the 1-hydroxyl group of 1D-myo-inositol.